{
  "term_id": "UNKNOWN:0002",
  "gene_name": "WD repeat-containing protein 90",
  "term_label": "Unknown biological process",
  "gene": "UniProtKB:Q96KV7",
  "gene_symbol": "WDR90"
}